{
  "gene_symbol": "ZNF66",
  "term_id": "GO:0000981",
  "term_label": "DNA-binding transcription factor activity, RNA polymerase II-specific",
  "gene_name": "Putative zinc finger protein 66",
  "gene": "UniProtKB:Q6ZN08"
}